{
  "term_label": "Unknown cellular component",
  "gene_name": "DNA oxidative demethylase ALKBH2",
  "gene": "UniProtKB:Q6NS38",
  "gene_symbol": "ALKBH2",
  "term_id": "UNKNOWN:0003"
}